mesonephric capsule formation [GO:0061287] (BP) Definition: The developmental process pertaining to the initial formation of a mesonephric capsule from unspecified parts. The mesonephric capsule is the tough fibrous layer surrounding the mesonephros, covered in a thick layer of perinephric adipose tissue. It provides some protection from trauma and damage. Sources: GOC:mtg_kidney_jan10 Relationships: is a type of GO:0072129; is part of mesonephric capsule morphogenesis [GO:0061286]